dAMP salvage [GO:0106383] (biological process) Relationships: is_a GO:0006170; is a type of GO:0106381 Definition: Any process which produces a dAMP from derivatives of it, without de novo synthesis. References: PMID:21829339, PMID:6605343